{
  "term_id": "UNKNOWN:0001",
  "gene_symbol": "DOCK8-AS1",
  "gene_name": "Uncharacterized protein DOCK8-AS1",
  "gene": "UniProtKB:Q5T8R8",
  "term_label": "Unknown molecular function"
}